{
  "gene_symbol": "ACTBL2",
  "gene_name": "Beta-actin-like protein 2",
  "term_label": "axonogenesis",
  "gene": "UniProtKB:Q562R1",
  "term_id": "GO:0007409"
}